{
  "gene": "UniProtKB:P11474",
  "term_id": "GO:0006357",
  "gene_name": "Steroid hormone receptor ERR1",
  "term_label": "regulation of transcription by RNA polymerase II",
  "gene_symbol": "ESRRA"
}